{
  "term_id": "GO:0045197",
  "gene": "UniProtKB:Q14160",
  "gene_symbol": "SCRIB",
  "term_label": "establishment or maintenance of epithelial cell apical/basal polarity",
  "gene_name": "Protein scribble homolog"
}